{
  "gene_name": "TSSK6-activating co-chaperone protein",
  "gene_symbol": "TSACC",
  "term_label": "cytoplasm",
  "gene": "UniProtKB:Q96A04",
  "term_id": "GO:0005737"
}